{
  "gene_symbol": "TOP3A",
  "term_label": "DNA recombination",
  "gene": "UniProtKB:Q13472",
  "gene_name": "DNA topoisomerase 3-alpha",
  "term_id": "GO:0006310"
}